adenylyltransferase activity [GO:0070566] (molecular function) Definition: Catalysis of the transfer of an adenylyl group to an acceptor. Subtypes: GO:0000309, GO:0001730, GO:0003877, FMN adenylyltransferase activity [GO:0003919], nicotinate-nucleotide adenylyltransferase activity [GO:0004515], pantetheine-phosphate adenylyltransferase activity [GO:0004595], GO:0004779, glucose-1-phosphate adenylyltransferase activity [GO:0008878], [glutamate-ammonia-ligase] adenylyltransferase activity [GO:0008882], GO:0033786, GO:0043910, GO:0047345, aldose-1-phosphate adenylyltransferase activity [GO:0047346], adenylylsulfate-ammonia adenylyltransferase activity [GO:0047352], ATP:3'-cytidine-cytidine-tRNA adenylyltransferase activity [GO:0052929], GO:0061598, molybdopterin-synthase adenylyltransferase activity [GO:0061605], AMPylase activity [GO:0070733], selenate adenylyltransferase (ATP) activity [GO:0098616], ATP:ATP adenylyltransferase activity [GO:0141192], poly(A) RNA polymerase activity [GO:1990817] Sources: GOC:mah Relationships: is a type of nucleotidyltransferase activity [GO:0016779]